hyaloid vascular plexus regression [GO:1990384] (biological process) References: PMID:18841878 Sources: GOC:hjd Relationships: is a type of GO:0060033; is part of camera-type eye development [GO:0043010] Definition: The developmental process in which the hyaloid vascular plexus is destroyed as a part of its normal progression.